{
  "term_label": "guanyl-nucleotide exchange factor activity",
  "term_id": "GO:0005085",
  "gene_name": "Dedicator of cytokinesis protein 2",
  "gene_symbol": "DOCK2",
  "gene": "UniProtKB:Q92608"
}